{
  "gene_symbol": "NEK2",
  "term_label": "chromosome segregation",
  "gene": "UniProtKB:P51955",
  "term_id": "GO:0007059",
  "gene_name": "Serine_threonine-protein kinase Nek2"
}